{
  "term_id": "GO:0006555",
  "term_label": "methionine metabolic process",
  "gene_name": "Acireductone dioxygenase",
  "gene_symbol": "ADI1",
  "gene": "UniProtKB:Q9BV57"
}